homogalacturonan metabolic process [GO:0010394] (biological process) Definition: The chemical reactions and pathways involving homogalacturonan, a pectin characterized by a backbone of alpha-(1->4)-linked D-galacturonic acid residues that can be methyl-esterified at C-6 and carry acetyl groups on O-2 and O-3. Subtypes: homogalacturonan biosynthetic process [GO:0010289], homogalacturonan catabolic process [GO:0033393] Also known as: homogalacturonan metabolism Sources: GOC:tair_curators Relationships: is a type of galacturonan metabolic process [GO:0010393]